{
  "gene_symbol": "VENTX",
  "gene": "UniProtKB:O95231",
  "term_label": "cell differentiation",
  "gene_name": "Homeobox protein VENTX",
  "term_id": "GO:0030154"
}